{
  "term_label": "positive regulation of tumor necrosis factor production",
  "gene_name": "Low affinity immunoglobulin gamma Fc region receptor II-a",
  "term_id": "GO:0032760",
  "gene": "UniProtKB:P12318",
  "gene_symbol": "FCGR2A"
}